{
  "term_id": "GO:0005179",
  "gene": "UniProtKB:Q4G0M1",
  "term_label": "hormone activity",
  "gene_name": "Erythroferrone",
  "gene_symbol": "ERFE"
}